{
  "term_label": "Unknown biological process",
  "term_id": "UNKNOWN:0002",
  "gene": "UniProtKB:A0A2R8YFM6",
  "gene_name": "Oocyte-secreted protein 3",
  "gene_symbol": "OOSP3"
}